{
  "term_id": "GO:0045087",
  "gene_symbol": "DEFB121",
  "term_label": "innate immune response",
  "gene": "UniProtKB:Q5J5C9",
  "gene_name": "Beta-defensin 121"
}